{
  "gene_symbol": "PRDM2",
  "term_id": "GO:0006357",
  "gene_name": "PR domain zinc finger protein 2",
  "gene": "UniProtKB:Q13029",
  "term_label": "regulation of transcription by RNA polymerase II"
}